{
  "gene": "UniProtKB:Q6SPF0",
  "term_id": "GO:0003682",
  "term_label": "chromatin binding",
  "gene_symbol": "SAMD1",
  "gene_name": "Sterile alpha motif domain-containing protein 1"
}